chemokine binding [GO:0019956] (molecular function) Definition: Binding to a chemokine. Chemokines are a family of small chemotactic cytokines; their name is derived from their ability to induce directed chemotaxis in nearby responsive cells. All chemokines possess a number of conserved cysteine residues involved in intramolecular disulfide bond formation. Some chemokines are considered pro-inflammatory and can be induced during an immune response to recruit cells of the immune system to a site of infection, while others are considered homeostatic and are involved in controlling the migration of cells during normal processes of tissue maintenance or development. Chemokines are found in all vertebrates, some viruses and some bacteria. References: PMID:12183377 Sources: GOC:BHF, GOC:ai, GOC:rl, Wikipedia:Chemokine Relationships: is a type of GO:0019955 Subtypes: C-C chemokine binding [GO:0019957], C-X-C chemokine binding [GO:0019958], C-X3-C chemokine binding [GO:0019960]